{
  "gene": "UniProtKB:O43795",
  "term_id": "GO:0051015",
  "term_label": "actin filament binding",
  "gene_name": "Unconventional myosin-Ib",
  "gene_symbol": "MYO1B"
}